{
  "gene_name": "1-phosphatidylinositol 4,5-bisphosphate phosphodiesterase eta-1",
  "gene": "UniProtKB:Q4KWH8",
  "gene_symbol": "PLCH1",
  "term_id": "GO:0051209",
  "term_label": "release of sequestered calcium ion into cytosol"
}